{
  "gene_name": "Serine palmitoyltransferase small subunit B",
  "gene_symbol": "SPTSSB",
  "term_id": "GO:0017059",
  "gene": "UniProtKB:Q8NFR3",
  "term_label": "serine palmitoyltransferase complex"
}